negative regulation of phosphatidylcholine catabolic process [GO:0010900] (biological process) Definition: Any process that decreases the rate, frequency or extent of phosphatidylcholine catabolism. Phosphatidylcholine catabolic processes are the chemical reactions and pathways resulting in the breakdown of phosphatidylcholines, any of a class of glycerophospholipids in which the phosphatidyl group is esterified to the hydroxyl group of choline. Sources: GOC:BHF, GOC:tb Relationships: is a type of regulation of phosphatidylcholine catabolic process [GO:0010899]; is a type of negative regulation of lipid catabolic process [GO:0050995]; is a type of GO:1903726; negatively regulates GO:0034638